{
  "gene": "UniProtKB:Q14696",
  "gene_symbol": "MESD",
  "term_label": "Unknown biological process",
  "gene_name": "LRP chaperone MESD",
  "term_id": "UNKNOWN:0002"
}